{
  "gene": "UniProtKB:O95264",
  "term_label": "transmembrane transporter complex",
  "gene_symbol": "HTR3B",
  "term_id": "GO:1902495",
  "gene_name": "5-hydroxytryptamine receptor 3B"
}